{
  "term_id": "GO:0004588",
  "gene": "UniProtKB:P11172",
  "term_label": "orotate phosphoribosyltransferase activity",
  "gene_symbol": "UMPS",
  "gene_name": "Uridine 5'-monophosphate synthase"
}